{
  "term_id": "UNKNOWN:0001",
  "gene_symbol": "PAGE2B",
  "gene_name": "Putative G antigen family E member 3",
  "term_label": "Unknown molecular function",
  "gene": "UniProtKB:Q5JRK9"
}